{
  "gene": "UniProtKB:P55285",
  "term_label": "cell morphogenesis",
  "gene_name": "Cadherin-6",
  "gene_symbol": "CDH6",
  "term_id": "GO:0000902"
}